{
  "gene_symbol": "ITGB1BP1",
  "term_label": "lamellipodium",
  "term_id": "GO:0030027",
  "gene_name": "Integrin beta-1-binding protein 1",
  "gene": "UniProtKB:O14713"
}